prenylated protein catabolic process [GO:0030327] (BP) Definition: The chemical reactions and pathways resulting in the breakdown of prenylated proteins. Sources: GOC:mah Also known as: prenylated protein breakdown, prenylated protein catabolism, prenylated protein degradation Relationships: is a type of modification-dependent protein catabolic process [GO:0019941]